{
  "term_id": "UNKNOWN:0003",
  "gene_name": "Peptidyl-prolyl cis-trans isomerase FKBP5",
  "gene": "UniProtKB:Q13451",
  "term_label": "Unknown cellular component",
  "gene_symbol": "FKBP5"
}